L-iditol 2-dehydrogenase (NAD+) activity [GO:0003939] (molecular function) References: PMID:13373783 Sources: EC:1.1.1.14 Also known as: polyol dehydrogenase activity, L-iditol (sorbitol) dehydrogenase activity, L-iditol:NAD oxidoreductase activity, L-iditol:NAD+ 5-oxidoreductase activity, NAD+-dependent sorbitol dehydrogenase activity, NAD-dependent sorbitol dehydrogenase activity, NAD-sorbitol dehydrogenase, glucitol dehydrogenase activity, sorbitol dehydrogenase activity Definition: Catalysis of the reaction: L-iditol + NAD+ = L-sorbose + NADH + H+. Acts on a number of sugar alcohols, including (but not limited to) L-iditol, D-glucitol, D-xylitol, and D-galactitol. Relationships: is_a alcohol dehydrogenase (NAD+) activity [GO:0004022]